{
  "gene": "UniProtKB:Q8N6T0",
  "gene_symbol": "TOP6BL",
  "gene_name": "Type 2 DNA topoisomerase 6 subunit B-like",
  "term_id": "UNKNOWN:0003",
  "term_label": "Unknown cellular component"
}